regulation of plant-type cell wall cellulose biosynthetic process [GO:2001009] (biological process) Relationships: is a type of regulation of cell wall macromolecule metabolic process [GO:0010981]; is a type of regulation of cellulose biosynthetic process [GO:2001006]; regulates plant-type cell wall cellulose biosynthetic process [GO:0052324] Definition: Any process that modulates the frequency, rate or extent of plant-type cell wall cellulose biosynthetic process. Sources: GOC:mengo_curators Subtypes: negative regulation of plant-type cell wall cellulose biosynthetic process [GO:2001010], GO:2001011 Also known as: regulation of cell wall cellulose biosynthesis, regulation of cellulose biosynthesis during cell wall biosynthesis